O antigen biosynthetic process [GO:0009243] (biological process) Sources: ISBN:0198506732 Also known as: O antigen anabolism, O antigen biosynthesis, O antigen formation, O antigen synthesis Relationships: is a type of GO:0000271; is part of lipopolysaccharide biosynthetic process [GO:0009103] Definition: The chemical reactions and pathways resulting in the formation of the O side chain of a lipopolysaccharide, which determines the antigenic specificity of the organism. It is made up of about 50 repeating units of a branched tetrasaccharide.